{
  "gene_symbol": "SLC38A3",
  "gene_name": "Sodium-coupled neutral amino acid transporter 3",
  "gene": "UniProtKB:Q99624",
  "term_label": "L-glutamine transmembrane transporter activity",
  "term_id": "GO:0015186"
}